{
  "term_label": "single-stranded DNA binding",
  "gene_symbol": "TWNK",
  "gene_name": "Twinkle mtDNA helicase",
  "term_id": "GO:0003697",
  "gene": "UniProtKB:Q96RR1"
}